spindle assembly involved in female meiosis I [GO:0007057] (biological process) Definition: The aggregation, arrangement and bonding together of a set of components to form the spindle during meiosis I of a meiotic cell cycle in females. An example of this is found in Drosophila melanogaster. Sources: GOC:mah Relationships: is a type of GO:0007056; is part of GO:0007144 Also known as: female meiosis I spindle assembly